{
  "gene_symbol": "SWT1",
  "term_id": "UNKNOWN:0002",
  "gene_name": "Transcriptional protein SWT1",
  "term_label": "Unknown biological process",
  "gene": "UniProtKB:Q5T5J6"
}